isoflavone 7-O-methyltransferase activity [GO:0033800] (molecular function) Sources: EC:2.1.1.150 Definition: Catalysis of the reaction: S-adenosyl-L-methionine + a 7-hydroxyisoflavone = S-adenosyl-L-homocysteine + a 7-methoxyisoflavone. Also known as: S-adenosyl-L-methionine:hydroxyisoflavone 7-O-methyltransferase activity Relationships: is a type of O-methyltransferase activity [GO:0008171]; is a type of S-adenosylmethionine-dependent methyltransferase activity [GO:0008757]